{
  "term_label": "Unknown biological process",
  "gene": "UniProtKB:Q8N319",
  "gene_symbol": "LINC03040",
  "term_id": "UNKNOWN:0002",
  "gene_name": "Putative uncharacterized protein encoded by LINC03040"
}